negative regulation of amyloid precursor protein catabolic process [GO:1902992] (biological process) Definition: Any process that stops, prevents or reduces the frequency, rate or extent of amyloid precursor protein catabolic process. References: PMID:24499793 Sources: GOC:PARL, GOC:TermGenie, GOC:rl, GO_REF:0000058 Also known as: down regulation of APP catabolic process, down regulation of APP catabolism, down regulation of amyloid precursor protein breakdown, down regulation of amyloid precursor protein catabolic process, down regulation of amyloid precursor protein catabolism, down regulation of amyloid precursor protein degradation, down-regulation of APP catabolic process, down-regulation of APP catabolism, down-regulation of amyloid precursor protein breakdown, down-regulation of amyloid precursor protein catabolic process, down-regulation of amyloid precursor protein catabolism, down-regulation of amyloid precursor protein degradation, downregulation of APP catabolic process, downregulation of APP catabolism, downregulation of amyloid precursor protein breakdown, downregulation of amyloid precursor protein catabolic process, downregulation of amyloid precursor protein catabolism, downregulation of amyloid precursor protein degradation, negative regulation of APP catabolic process, negative regulation of APP catabolism, negative regulation of amyloid precursor protein breakdown, negative regulation of amyloid precursor protein catabolism, negative regulation of amyloid precursor protein degradation, inhibition of APP catabolic process, inhibition of APP catabolism, inhibition of amyloid precursor protein breakdown, inhibition of amyloid precursor protein catabolic process, inhibition of amyloid precursor protein catabolism, inhibition of amyloid precursor protein degradation Subtypes: negative regulation of amyloid-beta formation [GO:1902430] Relationships: is a type of negative regulation of protein metabolic process [GO:0051248]; is a type of regulation of amyloid precursor protein catabolic process [GO:1902991]; negatively regulates amyloid precursor protein catabolic process [GO:0042987]